meiotic metaphase chromosome alignment [GO:0051311] (biological process) Sources: GOC:vw Relationships: is a type of metaphase chromosome alignment [GO:0051310]; is_a GO:1903046; is part of meiotic chromosome segregation [GO:0045132] Subtypes: meiotic metaphase I homologous chromosome alignment [GO:0043060], meiotic metaphase II chromosome alignment [GO:0043061] Definition: A chromosome localization process whereby chromosomes are positioned in a specific order and orientation at the metaphase plate (spindle equator), during meiotic chromosome segregation. This alignment ensures that each daughter cell will receive the correct number of chromosomes during cell division. Also known as: metaphase plate congression during meiosis